{
  "term_label": "synaptic vesicle membrane",
  "gene_name": "Phagosome assembly factor 1",
  "term_id": "GO:0030672",
  "gene_symbol": "PHAF1",
  "gene": "UniProtKB:Q9BSU1"
}